behavioral response to chemical pain [GO:0061366] (biological process) Relationships: is_a GO:0007635; is a type of behavioral response to pain [GO:0048266] Sources: GOC:dph Subtypes: behavioral response to acetic acid induced pain [GO:0061367], behavioral response to formalin induced pain [GO:0061368] Definition: Any process that results in a change in the behaviour of an organism as a result of a chemical pain stimulus.